{
  "gene_symbol": "GABRA5",
  "term_label": "dendrite membrane",
  "gene_name": "Gamma-aminobutyric acid receptor subunit alpha-5",
  "gene": "UniProtKB:P31644",
  "term_id": "GO:0032590"
}